{
  "gene_symbol": "FAM83B",
  "term_label": "protein kinase binding",
  "term_id": "GO:0019901",
  "gene_name": "Protein FAM83B",
  "gene": "UniProtKB:Q5T0W9"
}